{
  "term_id": "GO:0030943",
  "gene_symbol": "TOMM20L",
  "gene_name": "TOMM20-like protein 1",
  "gene": "UniProtKB:Q6UXN7",
  "term_label": "mitochondrion targeting sequence binding"
}